{
  "gene_symbol": "ANK1",
  "term_id": "GO:0008093",
  "gene": "UniProtKB:P16157",
  "term_label": "cytoskeletal anchor activity",
  "gene_name": "Ankyrin-1"
}